{
  "gene": "UniProtKB:Q9UN88",
  "gene_symbol": "GABRQ",
  "term_label": "GABA-A receptor complex",
  "gene_name": "Gamma-aminobutyric acid receptor subunit theta",
  "term_id": "GO:1902711"
}